{
  "gene_symbol": "IQCA1L",
  "term_id": "GO:0051013",
  "gene_name": "IQ and AAA domain-containing protein 1-like",
  "gene": "UniProtKB:A6NCM1",
  "term_label": "microtubule severing"
}